apical complex [GO:0020007] (cellular component) Definition: A group of cytoskeletal structures and associated membrane-bounded organelles found at the anterior end of adult obligate intracellular protozoan parasites in the phylum Apicomplexa. The apical complex is involved in attachment to and penetration of the host cell, and in parasite proliferation. References: PMID:16518471 Sources: GOC:giardia, GOC:mb Relationships: is_a cellular anatomical structure [GO:0110165]; BFO_0000050 apical part of cell [GO:0045177]